regulation of arbuscule formation for nutrient acquisition from host [GO:0075329] (biological process) Definition: Any process that modulates the frequency, rate or extent of symbiont arbuscule formation for nutrient acquisition from host. The host is defined as the larger of the organisms involved in a symbiotic interaction. Note: Note that this term should not be used to annotate gene products of the host. It should only be used to annotate those gene products from the symbiont involved in this process. Subtypes: positive regulation of arbuscule formation for nutrient acquisition from host [GO:0075330], negative regulation of arbuscule formation for nutrient acquisition from host [GO:0075331] Sources: GOC:pamgo_curators Relationships: is a type of regulation of anatomical structure morphogenesis [GO:0022603]; is a type of modulation of formation of structure involved in a symbiotic process [GO:0044145]; is a type of GO:0060259; RO_0002211 formation of arbuscule for nutrient acquisition [GO:0075328]